D-serine transmembrane transporter activity [GO:0042945] (molecular function) Definition: Enables the transfer of D-serine from one side of a membrane to the other. D-serine is the D-enantiomer of 2-amino-3-hydroxypropanoic acid. Sources: GOC:jl, GOC:jsg, GOC:mah, GOC:mtg_transport, ISBN:0815340729 Also known as: D-serine transporter activity, D-serine permease activity Relationships: is a type of D-amino acid transmembrane transporter activity [GO:0042943]; is part of D-serine transmembrane transport [GO:0042942]